3-hydroxy-2-methylquinolin-4-one 2,4-dioxygenase activity [GO:0050586] (molecular function) Definition: Catalysis of the reaction: 3-hydroxy-2-methylquinolin-4(1H)-one + H+ + O2 = N-acetylanthranilate + CO. Sources: EC:1.13.11.48, RHEA:21572 Also known as: 1H-3-hydroxy-4-oxo quinaldine 2,4-dioxygenase activity, 1H-3-hydroxy-4-oxoquinaldine 2,4-dioxygenase activity, 3-hydroxy-2-methyl-quinolin-4-one 2,4-dioxygenase activity, (1H)-3-hydroxy-4-oxoquinaldine 2,4-dioxygenase activity, 3-hydroxy-2-methyl-1H-quinolin-4-one 2,4-dioxygenase (CO-forming) Relationships: is a type of oxidoreductase activity, acting on single donors with incorporation of molecular oxygen, incorporation of two atoms of oxygen [GO:0016702]